{
  "gene_symbol": "SUN2",
  "term_label": "Unknown biological process",
  "term_id": "UNKNOWN:0002",
  "gene_name": "SUN domain-containing protein 2",
  "gene": "UniProtKB:Q9UH99"
}